{
  "term_id": "UNKNOWN:0001",
  "gene": "UniProtKB:O43633",
  "gene_symbol": "CHMP2A",
  "gene_name": "Charged multivesicular body protein 2a",
  "term_label": "Unknown molecular function"
}